enterocyte differentiation [GO:1903703] (biological process) Relationships: is a type of intestinal epithelial cell differentiation [GO:0060575] References: PMID:16782882 Sources: GOC:TermGenie, GO_REF:0000086, Wikipedia:List_of_intestinal_epithelial_differentiation_genes Definition: The process in which a relatively unspecialized cell acquires the specialized features of an enterocyte.